{
  "term_id": "GO:0007076",
  "gene_symbol": "NCAPG",
  "gene_name": "Condensin complex subunit 3",
  "term_label": "mitotic chromosome condensation",
  "gene": "UniProtKB:Q9BPX3"
}